post-embryonic ectodermal digestive tract morphogenesis [GO:0048614] (BP) Definition: The process, occurring during the post-embryonic phase, by which the anatomical structures of the ectodermal gut are generated and organized. Sources: GOC:jid, GOC:rc Also known as: post-embryonic ectodermal gut morphogenesis Relationships: is a type of post-embryonic animal morphogenesis [GO:0009886]; is part of GO:0048567; is part of GO:0048612; is part of post-embryonic digestive tract morphogenesis [GO:0048621]